{
  "term_id": "GO:0003924",
  "gene_name": "Septin-6",
  "gene": "UniProtKB:Q14141",
  "gene_symbol": "SEPTIN6",
  "term_label": "GTPase activity"
}